{
  "gene": "UniProtKB:O94762",
  "term_label": "nucleus",
  "term_id": "GO:0005634",
  "gene_symbol": "RECQL5",
  "gene_name": "ATP-dependent DNA helicase Q5"
}